GDP-galactose:glucose-1-phosphate guanylyltransferase activity [GO:0010472] (molecular function) Also known as: GDP-L-galactose phosphorylase activity, GDP-L-galactose:glucose-1-phosphate guanylyltransferase activity Relationships: is a type of guanylyltransferase activity [GO:0070568] References: PMID:17485667 Sources: RHEA:65712 Definition: Catalysis of the reaction: GDP-beta-L-galactose + alpha-D-glucose 1-phosphate = beta-L-galactose-1-phosphate + GDP-alpha-D-glucose.